acetyl-CoA synthetase acetyltransferase activity [GO:0043894] (molecular function) Relationships: is a type of acetyltransferase activity [GO:0016407] References: PMID:15236963 Definition: Catalysis of the acetylation of residue Lys609 of the enzyme acetyl-CoA synthetase, using acetyl-CoA as substrate. Also known as: protein acetyltransferase activity, Pat enzyme, Pat